{
  "gene_name": "G protein-regulated inducer of neurite outgrowth 1",
  "gene_symbol": "GPRIN1",
  "gene": "UniProtKB:Q7Z2K8",
  "term_id": "UNKNOWN:0001",
  "term_label": "Unknown molecular function"
}